positive regulation of meiotic DNA double-strand break formation [GO:1903343] (biological process) Subtypes: GO:1905263 Relationships: is a type of positive regulation of DNA metabolic process [GO:0051054]; is a type of positive regulation of cell cycle process [GO:0090068]; is_a regulation of meiotic DNA double-strand break formation [GO:1903341]; is a type of positive regulation of reproductive process [GO:2000243]; positively regulates GO:0042138 Also known as: up regulation of meiotic DNA double-strand break formation, up-regulation of meiotic DNA double-strand break formation, upregulation of meiotic DNA double-strand break formation, activation of meiotic DNA double-strand break formation Definition: Any process that activates or increases the frequency, rate or extent of meiotic DNA double-strand break formation. References: PMID:25103240 Sources: GOC:TermGenie, GO_REF:0000058